{
  "gene_symbol": "HPRT1",
  "gene_name": "Hypoxanthine-guanine phosphoribosyltransferase",
  "term_id": "GO:0005829",
  "term_label": "cytosol",
  "gene": "UniProtKB:P00492"
}